{
  "gene_name": "Guanine nucleotide-binding protein G(t) subunit alpha-2",
  "term_id": "GO:0001580",
  "gene_symbol": "GNAT2",
  "term_label": "detection of chemical stimulus involved in sensory perception of bitter taste",
  "gene": "UniProtKB:P19087"
}